{
  "term_id": "UNKNOWN:0003",
  "term_label": "Unknown cellular component",
  "gene_symbol": "CYBC1",
  "gene_name": "Cytochrome b-245 chaperone 1",
  "gene": "UniProtKB:Q9BQA9"
}